MAP kinase serine/threonine phosphatase activity [GO:1990439] (molecular function) Definition: Catalysis of the reaction: MAP kinase threonine phosphate + H2O = MAP kinase threonine + phosphate and MAP kinase serine phosphate + H2O = MAP kinase serine + phosphate. References: PMID:10398679 Relationships: is a type of protein serine/threonine phosphatase activity [GO:0004722]; is a type of MAP kinase phosphatase activity [GO:0033549]